{
  "gene_name": "Ubiquitin carboxyl-terminal hydrolase 28",
  "gene_symbol": "USP28",
  "term_id": "GO:0005829",
  "term_label": "cytosol",
  "gene": "UniProtKB:Q96RU2"
}